isochorismate synthase activity [GO:0008909] (MF) Sources: EC:5.4.4.2, RHEA:18985 Definition: Catalysis of the reaction: chorismate = isochorismate. Relationships: is a type of intramolecular hydroxytransferase activity [GO:0050486] Also known as: isochorismate mutase activity, isochorismate hydroxymutase activity, isochorismate synthetase activity